{
  "gene_symbol": "TBC1D12",
  "gene_name": "TBC1 domain family member 12",
  "term_label": "GTPase activator activity",
  "gene": "UniProtKB:O60347",
  "term_id": "GO:0005096"
}